secretion by the type IV secretion system [GO:0044097] (biological process) Also known as: secretion via the type IV secretion system Subtypes: GO:0030255, DNA secretion by the type IV secretion system [GO:0044098] Sources: GOC:pamgo_curators Definition: The controlled release of proteins or DNA by a cell, via the type IV secretion system. Relationships: is a type of secretion by cell [GO:0032940]